outer membrane protein complex [GO:0106234] (cellular component) Relationships: is a type of membrane protein complex [GO:0098796] References: PMID:25267629, PMID:27282389 Sources: GOC:am Definition: Any protein complex that is part of the bacterial outer membrane. An example In E.coli, is RcsF associated with any one of several outer membrane beta-barrel proteins (OMPs), such as OmpA, OmpF, or OmpcC.